regulation of T cell anergy [GO:0002667] (biological process) Subtypes: negative regulation of T cell anergy [GO:0002668], positive regulation of T cell anergy [GO:0002669] Sources: GOC:add Also known as: regulation of T lymphocyte anergy, regulation of T-cell anergy, regulation of T-lymphocyte anergy Relationships: is a type of regulation of T cell tolerance induction [GO:0002664]; is a type of regulation of lymphocyte anergy [GO:0002911]; regulates GO:0002870 Definition: Any process that modulates the frequency, rate, or extent of T cell anergy.